{
  "term_id": "UNKNOWN:0003",
  "gene_symbol": "SYCN",
  "term_label": "Unknown cellular component",
  "gene": "UniProtKB:Q0VAF6",
  "gene_name": "Syncollin"
}